{
  "gene": "UniProtKB:P46092",
  "term_label": "C-C chemokine binding",
  "gene_symbol": "CCR10",
  "gene_name": "C-C chemokine receptor type 10",
  "term_id": "GO:0019957"
}